cannabinoid receptor binding [GO:0031717] (molecular function) Subtypes: type 1 cannabinoid receptor binding [GO:0031718], type 2 cannabinoid receptor binding [GO:0031719] Definition: Binding to a cannabinoid receptor. Sources: GOC:mah, GOC:nln Relationships: is a type of G protein-coupled receptor binding [GO:0001664] Also known as: cannabinoid receptor ligand